{
  "term_id": "GO:0006355",
  "gene_name": "Zinc finger protein 488",
  "gene": "UniProtKB:Q96MN9",
  "term_label": "regulation of DNA-templated transcription",
  "gene_symbol": "ZNF488"
}